{
  "gene": "UniProtKB:P54750",
  "term_label": "calmodulin-activated 3',5'-cyclic-GMP phosphodiesterase activity",
  "gene_name": "Dual specificity calcium_calmodulin-dependent 3',5'-cyclic nucleotide phosphodiesterase 1A",
  "term_id": "GO:0048101",
  "gene_symbol": "PDE1A"
}